{
  "term_id": "GO:0030234",
  "gene": "UniProtKB:Q02221",
  "gene_symbol": "COX6A2",
  "term_label": "enzyme regulator activity",
  "gene_name": "Cytochrome c oxidase subunit 6A2, mitochondrial"
}